{
  "gene": "UniProtKB:P34972",
  "gene_name": "Cannabinoid receptor 2",
  "term_id": "GO:0004949",
  "term_label": "cannabinoid receptor activity",
  "gene_symbol": "CNR2"
}